{
  "term_label": "Unknown biological process",
  "gene_symbol": "TATDN3",
  "gene": "UniProtKB:Q17R31",
  "term_id": "UNKNOWN:0002",
  "gene_name": "Putative deoxyribonuclease TATDN3"
}